mimosinase activity [GO:0050101] (molecular function) Definition: Catalysis of the reaction: L-mimosine + H2O = 3-hydroxy-4H-pyrid-4-one + L-serine. Sources: GOC:curators, RHEA:75355 Also known as: mimosine amidohydrolase activity Relationships: is a type of GO:0016843